{
  "gene": "UniProtKB:Q8TDV2",
  "term_id": "GO:0050911",
  "gene_symbol": "GPR148",
  "gene_name": "Probable G-protein coupled receptor 148",
  "term_label": "detection of chemical stimulus involved in sensory perception of smell"
}